{
  "term_label": "L-asparagine transmembrane transporter activity",
  "gene_symbol": "SLC38A3",
  "gene_name": "Sodium-coupled neutral amino acid transporter 3",
  "gene": "UniProtKB:Q99624",
  "term_id": "GO:0015182"
}